early viral transcription [GO:0019085] (biological process) Relationships: is a type of viral transcription [GO:0019083] Also known as: immediate early viral mRNA transcription Definition: The first phase of viral transcription that occurs after entry of the virus into the host cell, but prior to viral genome replication. It involves the transcription of genes for non-structural proteins, and for lytic viruses, the early gene products are involved in establishing control over the host cell. Sources: GOC:bf, GOC:jh2, GOC:jl